{
  "term_id": "GO:0005634",
  "gene_symbol": "RORB",
  "gene": "UniProtKB:Q92753",
  "gene_name": "Nuclear receptor ROR-beta",
  "term_label": "nucleus"
}